{
  "gene_symbol": "MUC5B",
  "gene": "UniProtKB:Q9HC84",
  "gene_name": "Mucin-5B",
  "term_id": "GO:0031012",
  "term_label": "extracellular matrix"
}